{
  "gene": "UniProtKB:Q15572",
  "term_label": "fibrillar center",
  "term_id": "GO:0001650",
  "gene_symbol": "TAF1C",
  "gene_name": "TATA box-binding protein-associated factor RNA polymerase I subunit C"
}